{
  "gene_symbol": "TRIM64B",
  "gene_name": "Putative tripartite motif-containing protein 64B",
  "term_id": "GO:0045087",
  "term_label": "innate immune response",
  "gene": "UniProtKB:A6NI03"
}